{
  "gene_symbol": "OR10A5",
  "term_id": "GO:0005886",
  "term_label": "plasma membrane",
  "gene": "UniProtKB:Q9H207",
  "gene_name": "Olfactory receptor 10A5"
}